3-hydroxy-9,10-secoandrosta-1,3,5(10)-triene-9,17-dione monooxygenase activity [GO:0036383] (molecular function) Sources: EC:1.14.14.12, GOC:rs Relationships: is a type of oxidoreductase activity, acting on paired donors, with incorporation or reduction of molecular oxygen, reduced flavin or flavoprotein as one donor, and incorporation of one atom of oxygen [GO:0016712] Definition: Catalysis of the reaction: 3-hydroxy-9,10-secoandrosta-1,3,5(10)-triene-9,17-dione + FMNH2 + O2 = 3,4-dihydroxy-9,10-secoandrosta-1,3,5(10)-triene-9,17-dione + FMN + H2O.